{
  "term_id": "GO:0006357",
  "gene": "UniProtKB:P55318",
  "gene_name": "Hepatocyte nuclear factor 3-gamma",
  "gene_symbol": "FOXA3",
  "term_label": "regulation of transcription by RNA polymerase II"
}